{
  "gene_symbol": "HSPA14",
  "gene_name": "Heat shock 70 kDa protein 14",
  "term_label": "heat shock protein binding",
  "term_id": "GO:0031072",
  "gene": "UniProtKB:Q0VDF9"
}